triglyceride-rich lipoprotein particle remodeling [GO:0034370] (biological process) Relationships: is a type of GO:0034369 Definition: The acquisition, loss or modification of a protein or lipid within a triglyceride-rich lipoprotein particle, including the hydrolysis of triglyceride by lipoprotein lipase, with the subsequent loss of free fatty acid, and the transfer of cholesterol esters to a triglyceride-rich lipoprotein particle by cholesteryl ester transfer protein (CETP), with the simultaneous transfer of triglyceride from a triglyceride-rich lipoprotein particle. Sources: GOC:BHF, GOC:expert_pt, GOC:mah, GOC:rl Subtypes: GO:0034371, GO:0034372, GO:0034373 Also known as: triacylglycerol-rich lipoprotein particle remodeling, triacylglycerol-rich lipoprotein particle remodelling, triglyceride-rich lipoprotein particle remodelling